{
  "gene": "UniProtKB:Q96EY5",
  "gene_name": "Multivesicular body subunit 12A",
  "term_label": "ESCRT I complex",
  "gene_symbol": "MVB12A",
  "term_id": "GO:0000813"
}